{
  "term_label": "epoxygenase P450 pathway",
  "gene_name": "Cytochrome P450 2C8",
  "gene": "UniProtKB:P10632",
  "gene_symbol": "CYP2C8",
  "term_id": "GO:0019373"
}